{
  "term_label": "Unknown biological process",
  "gene": "UniProtKB:A1L157",
  "gene_symbol": "TSPAN11",
  "term_id": "UNKNOWN:0002",
  "gene_name": "Tetraspanin-11"
}